deuterosome [GO:0098536] (cellular component) Definition: A spherical, electron dense, cytoplasmic structure that is involved in de novo assembly of centrioles. References: PMID:24075808, PMID:25047614, PMID:5661997 Sources: GOC:cilia, GOC:dos Relationships: is a type of intracellular membraneless organelle [GO:0043232]